{
  "term_label": "coreceptor activity",
  "gene_name": "Receptor activity-modifying protein 1",
  "term_id": "GO:0015026",
  "gene": "UniProtKB:O60894",
  "gene_symbol": "RAMP1"
}